{
  "gene": "UniProtKB:Q8WWZ3",
  "term_label": "Unknown cellular component",
  "term_id": "UNKNOWN:0003",
  "gene_symbol": "EDARADD",
  "gene_name": "Ectodysplasin-A receptor-associated adapter protein"
}